{
  "term_id": "GO:0060090",
  "gene_symbol": "SEPTIN5",
  "gene": "UniProtKB:Q99719",
  "gene_name": "Septin-5",
  "term_label": "molecular adaptor activity"
}